{
  "gene_name": "Putative rhophilin-2-like protein RHPN2P1",
  "gene_symbol": "RHPN2P1",
  "term_label": "Unknown molecular function",
  "term_id": "UNKNOWN:0001",
  "gene": "UniProtKB:A8MT19"
}